arabinan metabolic process [GO:0031221] (biological process) Relationships: is_a polysaccharide metabolic process [GO:0005976] Subtypes: arabinan catabolic process [GO:0031222], arabinan biosynthetic process [GO:0035884] Sources: GOC:mlg, ISBN:0198506732 Definition: The chemical reactions and pathways involving arabinan, a polysaccharide composed of arabinose residues. Also known as: arabinan metabolism